{
  "gene_symbol": "ZCCHC18",
  "term_label": "Unknown molecular function",
  "gene": "UniProtKB:P0CG32",
  "gene_name": "Zinc finger CCHC domain-containing protein 18",
  "term_id": "UNKNOWN:0001"
}